{
  "gene_symbol": "SPSB3",
  "term_id": "GO:1990756",
  "term_label": "ubiquitin-like ligase-substrate adaptor activity",
  "gene_name": "SPRY domain-containing SOCS box protein 3",
  "gene": "UniProtKB:Q6PJ21"
}